voltage-gated potassium channel activity involved in cardiac muscle cell action potential repolarization [GO:0086008] (molecular function) Sources: GOC:BHF, GOC:mtg_cardiac_conduct_nov11 Relationships: is a type of voltage-gated potassium channel activity [GO:0005249]; is part of GO:0086013 Subtypes: voltage-gated potassium channel activity involved in AV node cell action potential repolarization [GO:0086086], GO:0086087, GO:0086088, voltage-gated potassium channel activity involved in atrial cardiac muscle cell action potential repolarization [GO:0086089], voltage-gated potassium channel activity involved in SA node cell action potential repolarization [GO:0086090], voltage-gated potassium channel activity involved in ventricular cardiac muscle cell action potential repolarization [GO:1902282] Definition: Enables the transmembrane transfer of a potassium ion by a voltage-gated channel through the plasma membrane of a cardiac muscle cell contributing to the repolarization phase of an action potential. A voltage-gated channel is a channel whose open state is dependent on the voltage across the membrane in which it is embedded.